{
  "gene": "UniProtKB:Q9Y5L4",
  "gene_symbol": "TIMM13",
  "term_id": "GO:0045039",
  "gene_name": "Mitochondrial import inner membrane translocase subunit Tim13",
  "term_label": "protein insertion into mitochondrial inner membrane"
}